{
  "term_id": "GO:0000981",
  "term_label": "DNA-binding transcription factor activity, RNA polymerase II-specific",
  "gene": "UniProtKB:Q9H4W6",
  "gene_name": "Transcription factor COE3",
  "gene_symbol": "EBF3"
}